{
  "gene_symbol": "DIS3L",
  "gene": "UniProtKB:Q8TF46",
  "gene_name": "DIS3-like exonuclease 1",
  "term_id": "GO:0016075",
  "term_label": "rRNA catabolic process"
}